cellular response to growth hormone stimulus [GO:0071378] (biological process) Definition: Any process that results in a change in state or activity of a cell (in terms of movement, secretion, enzyme production, gene expression, etc.) as a result of a growth hormone stimulus. Growth hormone is a peptide hormone that binds to the growth hormone receptor and stimulates growth. Sources: GOC:mah Relationships: is a type of response to growth hormone [GO:0060416]; is a type of cellular response to peptide hormone stimulus [GO:0071375]